{
  "gene_name": "Ribosomal protein eL22-like",
  "gene_symbol": "RPL22L1",
  "term_label": "RNA binding",
  "gene": "UniProtKB:Q6P5R6",
  "term_id": "GO:0003723"
}